galactose-specific flocculation [GO:0036349] (biological process) References: PMID:22098069 Sources: GOC:vw Definition: The non-sexual aggregation of single-celled organisms mediated by the binding of cell wall proteins on one cell to galactose residues on the other. Also known as: cell-cell adhesion involved in galactose-specific flocculation Relationships: is a type of flocculation [GO:0000128]; has part galactose binding [GO:0005534]